{
  "term_id": "GO:0004672",
  "term_label": "protein kinase activity",
  "gene_name": "Transient receptor potential cation channel subfamily M member 7",
  "gene": "UniProtKB:Q96QT4",
  "gene_symbol": "TRPM7"
}